{
  "term_id": "UNKNOWN:0001",
  "gene_symbol": "PRB1",
  "gene": "UniProtKB:P04280",
  "gene_name": "Basic salivary proline-rich protein 1",
  "term_label": "Unknown molecular function"
}